{
  "gene_name": "Early growth response protein 4",
  "gene_symbol": "EGR4",
  "term_id": "GO:0005634",
  "term_label": "nucleus",
  "gene": "UniProtKB:Q05215"
}